{
  "gene_symbol": "CC2D1A",
  "term_label": "regulation of transcription by RNA polymerase II",
  "term_id": "GO:0006357",
  "gene_name": "Coiled-coil and C2 domain-containing protein 1A",
  "gene": "UniProtKB:Q6P1N0"
}